de novo tRNA queuosine(34) biosynthetic process [GO:0160253] (biological process) References: PMID:28208705 Relationships: is a type of tRNA queuosine(34) biosynthetic process [GO:0008616] Definition: The chemical reactions and pathways resulting in the formation of tRNA queuosine(34) from guanosine triphosphate (GTP).